{
  "term_id": "GO:0005375",
  "term_label": "copper ion transmembrane transporter activity",
  "gene": "UniProtKB:O15431",
  "gene_symbol": "SLC31A1",
  "gene_name": "High affinity copper uptake protein 1"
}